pyrimidine ribonucleoside binding [GO:0032551] (molecular function) Definition: Binding to a pyrimidine ribonucleoside, a compound consisting of a pyrimidine base linked to ribose. Relationships: is a type of pyrimidine nucleoside binding [GO:0001884]; is a type of ribonucleoside binding [GO:0032549] Sources: GOC:mah